4,4'-diapophytoene desaturase (4,4'-diaponeurosporene-forming) [GO:0102223] (molecular function) References: PMID:8002598 Sources: RHEA:31391 Definition: Catalysis of the reaction: 4 H+ + 15-cis-4,4'-diapophytoene + 4 FAD = 4,4'-diapolycopene + 4 FADH2. This reaction consists of four successive dehydrogenations that lead to the introduction of three double bonds into 4,4'-diapophytoene (dehydrosqualene), with 4,4'-diapophytofluene, 4,4'-diapo-zeta-carotene and 4,4'-diapolycopene as intermediates, and 4,4'-diapolycopene as the end product. Also known as: 4,4'-diapophytoene desaturase activity, 4,4'-diapo-zeta-carotene desaturase activity, 4,4'-diaponeurosporene desaturase activity, 4,4'-diapophytofluene desaturase activity Relationships: is a type of oxidoreductase activity, acting on the CH-CH group of donors, with a flavin as acceptor [GO:0052890]